L-glutamate N-acetyltransferase activity, acting on acetyl-L-ornithine as donor [GO:0004358] (molecular function) Also known as: L-glutamate N-acetyltransferase activity, N-acetyl-L-glutamate synthetase activity, N-acetylglutamate synthase activity, N-acetylglutamate synthetase activity, acetylornithinase activity, glutamate N-acetyltransferase activity, acetyl-L-glutamate:acetyl-L-ornithine transacetylase activity, 2-N-acetyl-L-ornithine:L-glutamate N-acetyltransferase activity, N2-acetyl-L-ornithine:L-glutamate N-acetyltransferase activity, acetylglutamate synthetase activity, acetylglutamate-acetylornithine transacetylase activity, acetylglutamic synthetase activity, acetylglutamic-acetylornithine transacetylase activity, acetylornithine glutamate acetyltransferase activity, alpha-N-acetyl-L-ornithine:L-glutamate N-acetyltransferase activity, glutamate acetyltransferase activity, ornithine acetyltransferase activity, ornithine transacetylase activity Sources: RHEA:15349 Relationships: is a type of L-amino-acid N-acetyltransferase activity [GO:0140085] Definition: Catalysis of the reaction: N2-acetyl-L-ornithine + L-glutamate = N-acetyl-L-glutamate + L-ornithine.